{
  "gene": "UniProtKB:Q96NR7",
  "term_label": "Unknown cellular component",
  "gene_name": "Putative uncharacterized protein WWC2-AS2",
  "gene_symbol": "WWC2-AS2",
  "term_id": "UNKNOWN:0003"
}